{
  "gene": "UniProtKB:Q6AWC8",
  "term_id": "UNKNOWN:0003",
  "gene_name": "Putative uncharacterized protein LOC100129027",
  "term_label": "Unknown cellular component",
  "gene_symbol": "Q6AWC8"
}